ankyrin binding [GO:0030506] (molecular function) Sources: GOC:mah, ISBN:0198506732 Definition: Binding to ankyrin, a 200 kDa cytoskeletal protein that attaches other cytoskeletal proteins to integral membrane proteins. Relationships: is a type of cytoskeletal protein binding [GO:0008092]